regulation of myosin II filament organization [GO:0043519] (BP) Relationships: is a type of regulation of actin cytoskeleton organization [GO:0032956]; is a type of regulation of supramolecular fiber organization [GO:1902903]; regulates myosin II filament organization [GO:0031038] Subtypes: regulation of myosin II filament assembly [GO:0043520], regulation of myosin II filament disassembly [GO:0043521], GO:1904900, positive regulation of myosin II filament organization [GO:1904901] Sources: GOC:jl Definition: Any process that modulates the frequency, rate or extent of the assembly, arrangement of constituent parts, or disassembly of a bipolar filament composed of myosin II molecules. Also known as: regulation of myosin II filament organisation, regulation of myosin II filament assembly or disassembly